{
  "gene_symbol": "ELMO2",
  "gene": "UniProtKB:Q96JJ3",
  "gene_name": "Engulfment and cell motility protein 2",
  "term_label": "actin filament organization",
  "term_id": "GO:0007015"
}